coronary artery morphogenesis [GO:0060982] (biological process) Relationships: is a type of artery morphogenesis [GO:0048844]; is a type of coronary vasculature morphogenesis [GO:0060977] Sources: GOC:mtg_heart Definition: The process in which the anatomical structures of coronary arteries are generated and organized. Coronary arteries are blood vessels that transport blood to the heart muscle.